{
  "gene_symbol": "ITGA3",
  "term_label": "cell-cell adhesion",
  "gene": "UniProtKB:P26006",
  "term_id": "GO:0098609",
  "gene_name": "Integrin alpha-3"
}